{
  "term_id": "GO:0034185",
  "term_label": "apolipoprotein binding",
  "gene": "UniProtKB:P11150",
  "gene_name": "Hepatic triacylglycerol lipase",
  "gene_symbol": "LIPC"
}